{
  "term_label": "Unknown molecular function",
  "term_id": "UNKNOWN:0001",
  "gene": "UniProtKB:Q15819",
  "gene_name": "Ubiquitin-conjugating enzyme E2 variant 2",
  "gene_symbol": "UBE2V2"
}